{
  "term_label": "protein serine/threonine kinase activity",
  "gene_name": "Dual specificity testis-specific protein kinase 1",
  "gene_symbol": "TESK1",
  "gene": "UniProtKB:Q15569",
  "term_id": "GO:0004674"
}